{
  "term_id": "GO:0030125",
  "gene_name": "Adaptin ear-binding coat-associated protein 2",
  "term_label": "clathrin vesicle coat",
  "gene_symbol": "NECAP2",
  "gene": "UniProtKB:Q9NVZ3"
}